{
  "gene_name": "Caspase recruitment domain-containing protein 19",
  "gene": "UniProtKB:Q96LW7",
  "gene_symbol": "CARD19",
  "term_id": "UNKNOWN:0001",
  "term_label": "Unknown molecular function"
}